{
  "gene": "UniProtKB:P42684",
  "gene_name": "Tyrosine-protein kinase ABL2",
  "gene_symbol": "ABL2",
  "term_label": "plasma membrane",
  "term_id": "GO:0005886"
}